{
  "gene_symbol": "ZNRD2",
  "gene": "UniProtKB:O60232",
  "term_id": "UNKNOWN:0001",
  "gene_name": "Protein ZNRD2",
  "term_label": "Unknown molecular function"
}